{
  "term_label": "trans-Golgi network",
  "gene_symbol": "MARCHF9",
  "gene_name": "E3 ubiquitin-protein ligase MARCHF9",
  "gene": "UniProtKB:Q86YJ5",
  "term_id": "GO:0005802"
}